nose morphogenesis [GO:0043585] (biological process) Sources: GOC:jl Also known as: nasus morphogenesis Relationships: is_a sensory organ morphogenesis [GO:0090596]; is part of GO:0043584 Definition: The process in which the anatomical structures of the nose are generated and organized. The nose is the specialized structure of the face that serves as the organ of the sense of smell and as part of the respiratory system. Includes the nasi externus (external nose) and cavitas nasi (nasal cavity).